{
  "gene_symbol": "ROBO4",
  "term_id": "GO:0007156",
  "gene": "UniProtKB:Q8WZ75",
  "gene_name": "Roundabout homolog 4",
  "term_label": "homophilic cell-cell adhesion"
}